{
  "gene_symbol": "INS",
  "term_id": "GO:0005158",
  "term_label": "insulin receptor binding",
  "gene_name": "Insulin",
  "gene": "UniProtKB:P01308"
}